{
  "term_label": "structural constituent of postsynaptic actin cytoskeleton",
  "term_id": "GO:0098973",
  "gene_name": "POTE ankyrin domain family member E",
  "gene": "UniProtKB:Q6S8J3",
  "gene_symbol": "POTEE"
}